spinothalamic tract morphogenesis [GO:0021963] (BP) Definition: Generation of a long process of a CNS neuron, that carries efferent (outgoing) action potentials from the cell body in the spinal cord towards target cells in the thalamus. This axonal process is a member of those that make up the spinothalamic tract, one of the major routes of nociceptive signaling. Sources: GOC:cls, GOC:dgh, GOC:dph, GOC:jid, GO_REF:0000021 Relationships: is a type of central nervous system projection neuron axonogenesis [GO:0021952] Also known as: dorsolateral tract of Lissauer morphogenesis